{
  "gene_name": "Stimulator of interferon genes protein",
  "term_id": "GO:0051607",
  "gene_symbol": "STING1",
  "gene": "UniProtKB:Q86WV6",
  "term_label": "defense response to virus"
}